heart valve formation [GO:0003188] (biological process) Definition: The developmental process pertaining to the initial formation of a heart valve from unspecified parts. This process begins with the specific processes that contribute to the appearance of the discrete structure and ends when the structural rudiment is recognizable. Relationships: is a type of GO:0048646; is part of GO:0003179 Sources: GOC:mtg_heart Subtypes: aortic valve formation [GO:0003189], atrioventricular valve formation [GO:0003190], coronary sinus valve formation [GO:0003191], pulmonary valve formation [GO:0003193], sinoatrial valve formation [GO:0003194], ventriculo bulbo valve formation [GO:0003196]